{
  "gene": "UniProtKB:Q9H0R8",
  "gene_name": "Gamma-aminobutyric acid receptor-associated protein-like 1",
  "term_label": "autophagosome assembly",
  "term_id": "GO:0000045",
  "gene_symbol": "GABARAPL1"
}